{
  "term_id": "GO:0070776",
  "term_label": "MOZ/MORF histone acetyltransferase complex",
  "gene_symbol": "KAT6A",
  "gene": "UniProtKB:Q92794",
  "gene_name": "Histone acetyltransferase KAT6A"
}